{
  "gene": "UniProtKB:P47872",
  "gene_symbol": "SCTR",
  "term_id": "GO:0017046",
  "gene_name": "Secretin receptor",
  "term_label": "peptide hormone binding"
}